{
  "gene": "UniProtKB:Q9ULC8",
  "term_id": "GO:0005794",
  "gene_symbol": "ZDHHC8",
  "gene_name": "Palmitoyltransferase ZDHHC8",
  "term_label": "Golgi apparatus"
}